{
  "gene_symbol": "STAR",
  "term_label": "Unknown cellular component",
  "term_id": "UNKNOWN:0003",
  "gene": "UniProtKB:P49675",
  "gene_name": "Steroidogenic acute regulatory protein, mitochondrial"
}